{
  "gene_symbol": "LRRTM3",
  "term_label": "signaling receptor activity",
  "gene": "UniProtKB:Q86VH5",
  "term_id": "GO:0038023",
  "gene_name": "Leucine-rich repeat transmembrane neuronal protein 3"
}